{
  "gene_symbol": "PER3",
  "term_id": "GO:0005737",
  "term_label": "cytoplasm",
  "gene": "UniProtKB:P56645",
  "gene_name": "Period circadian protein homolog 3"
}